{
  "gene": "UniProtKB:B1AK76",
  "gene_name": "Putative SNURF-like protein",
  "gene_symbol": "SNURFL",
  "term_label": "Unknown biological process",
  "term_id": "UNKNOWN:0002"
}